{
  "term_label": "phospholipid transport",
  "gene_symbol": "OSBPL5",
  "gene": "UniProtKB:Q9H0X9",
  "gene_name": "Oxysterol-binding protein-related protein 5",
  "term_id": "GO:0015914"
}